hepatocyte dedifferentiation [GO:1990828] (biological process) Definition: The process in which a hepatocyte (specialized epithelial cell of the liver) loses the structural or functional features that characterize it in the mature organism, or some other relatively stable phase of the organism's life history. Under certain conditions, these cells can revert back to the features of the stem cells that were their ancestors. Relationships: is a type of cell dedifferentiation [GO:0043697] References: PMID:20102719